{
  "term_id": "UNKNOWN:0003",
  "gene_name": "Uncharacterized protein FLJ40521",
  "gene_symbol": "Q8N7P7",
  "gene": "UniProtKB:Q8N7P7",
  "term_label": "Unknown cellular component"
}